{
  "term_id": "GO:0006405",
  "gene_name": "mRNA export factor RAE1",
  "gene_symbol": "RAE1",
  "term_label": "RNA export from nucleus",
  "gene": "UniProtKB:P78406"
}